{
  "gene": "UniProtKB:O60687",
  "gene_name": "Sushi repeat-containing protein SRPX2",
  "term_label": "positive regulation of cell migration involved in sprouting angiogenesis",
  "term_id": "GO:0090050",
  "gene_symbol": "SRPX2"
}